{
  "gene": "UniProtKB:A0A075B767",
  "term_label": "cyclosporin A binding",
  "gene_symbol": "PPIAL4H",
  "gene_name": "Peptidyl-prolyl cis-trans isomerase A-like 4H",
  "term_id": "GO:0016018"
}